high molecular weight kininogen binding [GO:0030985] (molecular function) Relationships: is a type of kininogen binding [GO:0030984] Definition: Binding to a kininogen of high molecular mass. Also known as: HK binding, HMW kininogen binding References: PMID:9520414 Sources: GOC:mah